establishment of protein localization to T cell secretory granule [GO:0033376] (biological process) Also known as: establishment of protein localisation in T cell secretory granule, establishment of protein localization in T cell secretory granule, establishment of protein localization in T lymphocyte secretory granule, establishment of protein localization in T-cell secretory granule, establishment of protein localization in T-lymphocyte secretory granule Relationships: is a type of GO:0006886; is part of GO:0033374 Sources: GOC:mah Definition: The directed movement of a protein to a location within a secretory granule in a T cell. Subtypes: establishment of protease localization to T cell secretory granule [GO:0033378]